{
  "gene": "UniProtKB:Q6IQ55",
  "gene_name": "Tau-tubulin kinase 2",
  "term_label": "ciliary basal body",
  "gene_symbol": "TTBK2",
  "term_id": "GO:0036064"
}